synaptic vesicle [GO:0008021] (cellular component) Relationships: is a type of exocytic vesicle [GO:0070382]; is part of presynapse [GO:0098793] References: PMID:10099709, PMID:12563290 Subtypes: GO:1990474, GO:1990475, GO:1990476 Note: This term should not be confused with GO:0097547 'synaptic vesicle protein transport vesicle'. STVs and synaptic vesicles differ both functionally and morphologically. Functionally, STVs are transport vesicles that deliver synaptic vesicle proteins to synapses, while synaptic vesicles are responsible for transmitter release at synapses. Morphologically, synaptic vesicles are very homogeneous, while STVs are very heterogeneous in size and shape. STVs might be a precursor for synaptic vesicles. Also known as: docked vesicle Definition: A secretory organelle, typically 50 nm in diameter, of presynaptic nerve terminals; accumulates in high concentrations of neurotransmitters and secretes these into the synaptic cleft by fusion with the 'active zone' of the presynaptic plasma membrane.